{
  "term_label": "actin cytoskeleton",
  "gene_symbol": "MYO1A",
  "term_id": "GO:0015629",
  "gene": "UniProtKB:Q9UBC5",
  "gene_name": "Unconventional myosin-Ia"
}